{
  "gene": "UniProtKB:Q96F44",
  "gene_symbol": "TRIM11",
  "term_id": "GO:0010468",
  "gene_name": "E3 ubiquitin-protein ligase TRIM11",
  "term_label": "regulation of gene expression"
}